regulation of nervous system development [GO:0051960] (biological process) Subtypes: GO:0031641, regulation of neurogenesis [GO:0050767], negative regulation of nervous system development [GO:0051961], GO:0051962 Relationships: is a type of regulation of multicellular organismal development [GO:2000026]; regulates nervous system development [GO:0007399] Sources: GOC:ai Definition: Any process that modulates the frequency, rate or extent of nervous system development, the origin and formation of nervous tissue.